{
  "term_label": "nucleus",
  "gene": "UniProtKB:Q9UL49",
  "term_id": "GO:0005634",
  "gene_name": "Transcription factor-like 5 protein",
  "gene_symbol": "TCFL5"
}